{
  "gene_symbol": "ALPK2",
  "term_id": "UNKNOWN:0003",
  "gene_name": "Alpha-protein kinase 2",
  "gene": "UniProtKB:Q86TB3",
  "term_label": "Unknown cellular component"
}